{
  "gene_symbol": "FAM201A",
  "term_label": "Unknown cellular component",
  "term_id": "UNKNOWN:0003",
  "gene": "UniProtKB:Q5SY85",
  "gene_name": "Protein FAM201A"
}